{
  "gene_name": "Equilibrative nucleoside transporter 3",
  "term_label": "nucleoside transmembrane transporter activity",
  "gene_symbol": "SLC29A3",
  "term_id": "GO:0005337",
  "gene": "UniProtKB:Q9BZD2"
}